{
  "term_label": "positive regulation of tumor necrosis factor production",
  "term_id": "GO:0032760",
  "gene": "UniProtKB:P31994",
  "gene_symbol": "FCGR2B",
  "gene_name": "Low affinity immunoglobulin gamma Fc region receptor II-b"
}